{
  "gene_symbol": "KITLG",
  "gene_name": "Kit ligand",
  "term_id": "GO:0005125",
  "gene": "UniProtKB:P21583",
  "term_label": "cytokine activity"
}